acetate:proton symporter activity [GO:0015360] (molecular function) Sources: TC:2.A.44.4.1 Definition: Enables the transfer of a solute or solutes from one side of a membrane to the other according to the reaction: acetate(out) + H+(out) = acetate(in) + H+(in). Relationships: is a type of solute:proton symporter activity [GO:0015295]; is a type of acetate:monoatomic cation symporter activity [GO:0043893] Also known as: acetate:hydrogen symporter activity, hydrogen:acetate symporter activity